{
  "gene": "UniProtKB:Q96J65",
  "gene_symbol": "ABCC12",
  "term_label": "ABC-type transporter activity",
  "term_id": "GO:0140359",
  "gene_name": "ATP-binding cassette sub-family C member 12"
}